rhombomere 2 formation [GO:0021657] (biological process) Definition: The process that gives rise to rhombomere 2. This process pertains to the initial formation of a structure from unspecified parts. Rhombomeres are transverse segments of the developing rhombencephalon. Rhombomeres are lineage restricted, express different genes from one another, and adopt different developmental fates. Rhombomeres are numbered in anterior to posterior order. Relationships: is a type of rhombomere formation [GO:0021594]; is part of GO:0021655 Sources: GOC:cls, GOC:curators, GOC:dgh, GOC:dph, GOC:jid